{
  "term_label": "deNEDDylase activity",
  "gene": "UniProtKB:Q96LD8",
  "term_id": "GO:0019784",
  "gene_symbol": "SENP8",
  "gene_name": "Sentrin-specific protease 8"
}